{
  "gene": "UniProtKB:Q8WVJ9",
  "gene_symbol": "TWIST2",
  "term_label": "RNA polymerase II transcription regulatory region sequence-specific DNA binding",
  "gene_name": "Twist-related protein 2",
  "term_id": "GO:0000977"
}